{
  "gene_name": "DAZ-associated protein 2",
  "gene_symbol": "DAZAP2",
  "term_label": "Unknown molecular function",
  "gene": "UniProtKB:Q15038",
  "term_id": "UNKNOWN:0001"
}